steviolmonoside glucosyltransferase activity [GO:0102378] (molecular function) Relationships: is a type of hexosyltransferase activity [GO:0016758] Definition: Catalysis of the reaction: steviolmonoside + UDP-alpha-D-glucose = rubusoside + UDP. Sources: RHEA:61736